iron-sulfur-molybdenum cofactor catabolic process [GO:1901287] (biological process) Also known as: FeMo-co breakdown, FeMo-co catabolic process, FeMo-co catabolism, FeMo-co degradation, iron-molybdenum breakdown, iron-molybdenum catabolic process, iron-molybdenum catabolism, iron-molybdenum degradation, iron-sulfur-molybdenum cofactor breakdown, iron-sulfur-molybdenum cofactor catabolism, iron-sulfur-molybdenum cofactor degradation Sources: GOC:TermGenie, GOC:yaf, UniPathway:UPA00782 Definition: The chemical reactions and pathways resulting in the breakdown of iron-sulfur-molybdenum cofactor. Relationships: is a type of catabolic process [GO:0009056]; is_a iron-sulfur-molybdenum cofactor metabolic process [GO:1901286]